astrocyte chemotaxis [GO:0035700] (biological process) Regulation: regulated by regulation of astrocyte chemotaxis [GO:2000458]; negatively regulated by negative regulation of astrocyte chemotaxis [GO:2000459]; RO_0002213 by positive regulation of astrocyte chemotaxis [GO:2000464] Definition: The directed movement of an astrocyte guided by a specific chemical concentration gradient. Movement may be towards a higher concentration (positive chemotaxis) or towards a lower concentration (negative chemotaxis). References: PMID:12271471 Sources: CL:0000127, GOC:BHF Relationships: is a type of astrocyte cell migration [GO:0043615]; is a type of GO:0060326